{
  "gene_name": "Leukocyte immunoglobulin-like receptor subfamily A member 4",
  "gene": "UniProtKB:P59901",
  "term_label": "plasma membrane",
  "term_id": "GO:0005886",
  "gene_symbol": "LILRA4"
}